{
  "gene_name": "UDP-glucuronosyltransferase 1A7",
  "gene_symbol": "UGT1A7",
  "gene": "UniProtKB:Q9HAW7",
  "term_label": "estrogen metabolic process",
  "term_id": "GO:0008210"
}